cellular response to blue light [GO:0071483] (biological process) Subtypes: blue light signaling pathway [GO:0009785] Definition: Any process that results in a change in state or activity of a cell (in terms of movement, secretion, enzyme production, gene expression, etc.) as a result of a blue light stimulus. Blue light is electromagnetic radiation with a wavelength of between 440 and 500nm. Relationships: is a type of response to blue light [GO:0009637]; is a type of cellular response to light stimulus [GO:0071482] Also known as: cellular response to blue light stimulus Sources: GOC:mah